{
  "gene": "UniProtKB:Q5SVS4",
  "gene_name": "Kidney mitochondrial carrier protein 1",
  "term_id": "GO:0022857",
  "gene_symbol": "SLC25A30",
  "term_label": "transmembrane transporter activity"
}